{
  "gene_name": "Dolichyldiphosphatase 1",
  "gene_symbol": "DOLPP1",
  "term_id": "GO:0006487",
  "gene": "UniProtKB:Q86YN1",
  "term_label": "protein N-linked glycosylation"
}